{
  "gene_name": "RNA binding protein fox-1 homolog 2",
  "gene": "UniProtKB:O43251",
  "term_label": "cytoplasm",
  "gene_symbol": "RBFOX2",
  "term_id": "GO:0005737"
}